{
  "gene_symbol": "CTSL",
  "gene_name": "Procathepsin L",
  "term_id": "GO:0005764",
  "gene": "UniProtKB:P07711",
  "term_label": "lysosome"
}